calcium ion transmembrane transport via high voltage-gated calcium channel [GO:0061577] (biological process) Also known as: generation of L-type calcium current Sources: GOC:dph Relationships: is a type of calcium ion transmembrane transport [GO:0070588]; has part high voltage-gated calcium channel activity [GO:0008331] Regulation: regulated by regulation of calcium ion transmembrane transport via high voltage-gated calcium channel [GO:1902514]; negatively regulated by negative regulation of calcium ion transmembrane transport via high voltage-gated calcium channel [GO:1904878]; positively regulated by GO:1904879 Definition: A process in which a calcium ion is transported from one side of a membrane to the other by means of a high voltage-gated calcium channel.